{
  "term_label": "actin filament binding",
  "gene": "UniProtKB:A7E2Y1",
  "gene_symbol": "MYH7B",
  "term_id": "GO:0051015",
  "gene_name": "Myosin-7B"
}